{
  "term_label": "plasma membrane",
  "term_id": "GO:0005886",
  "gene": "UniProtKB:Q9NUL3",
  "gene_symbol": "STAU2",
  "gene_name": "Double-stranded RNA-binding protein Staufen homolog 2"
}